cellular response to stem cell factor stimulus [GO:0036216] (biological process) Also known as: cellular response to KIT ligand, cellular response to KITLG, cellular response to SCF, cellular response to hematopoietic growth factor KL Definition: Any process that results in a change in state or activity of a cell (in terms of movement, secretion, enzyme production, gene expression, etc.) as a result of a stem cell factor (SCF) stimulus. References: PMID:18787413, PMID:7520444 Sources: GOC:uh Relationships: is a type of response to stem cell factor [GO:0036215]; is a type of cellular response to cytokine stimulus [GO:0071345]